{
  "term_label": "extracellular space",
  "gene_name": "Kallikrein-9",
  "gene": "UniProtKB:Q9UKQ9",
  "term_id": "GO:0005615",
  "gene_symbol": "KLK9"
}